{
  "term_label": "heme biosynthetic process",
  "gene": "UniProtKB:P22830",
  "gene_symbol": "FECH",
  "gene_name": "Ferrochelatase, mitochondrial",
  "term_id": "GO:0006783"
}